{
  "term_id": "GO:0005634",
  "gene_symbol": "GMEB2",
  "gene": "UniProtKB:Q9UKD1",
  "term_label": "nucleus",
  "gene_name": "Glucocorticoid modulatory element-binding protein 2"
}